{
  "gene": "UniProtKB:P51790",
  "gene_symbol": "CLCN3",
  "gene_name": "H(+)_Cl(-) exchange transporter 3",
  "term_id": "UNKNOWN:0002",
  "term_label": "Unknown biological process"
}